extrinsic component of matrix side of mitochondrial inner membrane [GO:0099616] (cellular component) Relationships: is a type of extrinsic component of mitochondrial inner membrane [GO:0031314]; is part of GO:0099617 Definition: The component of the matrix side of the mitochondrial inner membrane consisting of gene products and protein complexes that are loosely bound to one of its surfaces, but not integrated into the hydrophobic region. Sources: GOC:dos